{
  "gene": "UniProtKB:Q8N4P6",
  "gene_name": "Leucine-rich repeat-containing protein 71",
  "gene_symbol": "LRRC71",
  "term_id": "UNKNOWN:0001",
  "term_label": "Unknown molecular function"
}